{
  "term_id": "GO:0009897",
  "gene": "UniProtKB:P32246",
  "gene_symbol": "CCR1",
  "gene_name": "C-C chemokine receptor type 1",
  "term_label": "external side of plasma membrane"
}